{
  "gene_name": "Serine_threonine-protein phosphatase 2A 56 kDa regulatory subunit delta isoform",
  "term_label": "cytosol",
  "gene_symbol": "PPP2R5D",
  "term_id": "GO:0005829",
  "gene": "UniProtKB:Q14738"
}